phosphomethylpyrimidine synthase activity [GO:0070284] (molecular function) References: PMID:18953358 Sources: RHEA:24840 Definition: Catalysis of the reaction: 5-amino-1-(5-phospho-beta-D-ribosyl)imidazole + S-adenosyl-L-methionine = 4-amino-2-methyl-5-(phosphooxymethyl)pyrimidine + CO + 5'-deoxyadenosine + formate + L-methionine + 3 H+. Relationships: is a type of carbon-carbon lyase activity [GO:0016830] Also known as: 4-amino-5-hydroxymethyl-2-methylpyrimidine phosphate synthase activity, HMP-P synthase activity, ThiC